{
  "gene_symbol": "ZSCAN32",
  "term_id": "GO:0000978",
  "term_label": "RNA polymerase II cis-regulatory region sequence-specific DNA binding",
  "gene_name": "Zinc finger and SCAN domain-containing protein 32",
  "gene": "UniProtKB:Q9NX65"
}